spiracle morphogenesis, open tracheal system [GO:0035277] (biological process) Relationships: is a type of anatomical structure morphogenesis [GO:0009653]; is part of GO:0007424 Definition: The process in which the anatomical structures of a spiracle are generated and organized. Spiracles are the openings in the insect open tracheal system; externally they connect to the epidermis and internally they connect to the tracheal trunk. Also known as: spiracle morphogenesis References: PMID:10491268 Sources: GOC:mtg_sensu